Hsp27 protein binding [GO:0051008] (molecular function) Relationships: is a type of heat shock protein binding [GO:0031072] Sources: GOC:ai Definition: Binding to Hsp27 proteins, a lightweight heat shock protein.